{
  "gene": "UniProtKB:P98171",
  "term_id": "GO:0005737",
  "gene_symbol": "ARHGAP4",
  "term_label": "cytoplasm",
  "gene_name": "Rho GTPase-activating protein 4"
}